{
  "term_id": "GO:1901981",
  "gene_symbol": "SNX20",
  "gene_name": "Sorting nexin-20",
  "term_label": "phosphatidylinositol phosphate binding",
  "gene": "UniProtKB:Q7Z614"
}